{
  "gene_symbol": "SLC27A5",
  "term_id": "GO:0005886",
  "term_label": "plasma membrane",
  "gene": "UniProtKB:Q9Y2P5",
  "gene_name": "Long-chain fatty acid transport protein 5"
}